{
  "gene": "UniProtKB:P04181",
  "term_id": "GO:0004587",
  "term_label": "ornithine aminotransferase activity",
  "gene_symbol": "OAT",
  "gene_name": "Ornithine aminotransferase, mitochondrial"
}